{
  "gene": "UniProtKB:Q8WXS8",
  "term_label": "metalloendopeptidase activity",
  "term_id": "GO:0004222",
  "gene_symbol": "ADAMTS14",
  "gene_name": "A disintegrin and metalloproteinase with thrombospondin motifs 14"
}